{
  "term_id": "GO:2000562",
  "term_label": "negative regulation of CD4-positive, alpha-beta T cell proliferation",
  "gene_name": "Galectin-9",
  "gene": "UniProtKB:O00182",
  "gene_symbol": "LGALS9"
}